positive regulation of T-helper 1 cell cytokine production [GO:2000556] (biological process) Relationships: is a type of GO:0002726; is a type of GO:0002827; is a type of regulation of T-helper 1 cell cytokine production [GO:2000554]; RO_0002213 T-helper 1 cell cytokine production [GO:0035744] Definition: Any process that activates or increases the frequency, rate or extent of T-helper 1 cell cytokine production. Sources: GOC:obol Also known as: positive regulation of Th1 cell cytokine production